{
  "gene_name": "Rho guanine nucleotide exchange factor 33",
  "gene": "UniProtKB:A8MVX0",
  "gene_symbol": "ARHGEF33",
  "term_id": "UNKNOWN:0002",
  "term_label": "Unknown biological process"
}